{
  "gene_name": "TATA element modulatory factor",
  "gene_symbol": "TMF1",
  "term_label": "Unknown molecular function",
  "term_id": "UNKNOWN:0001",
  "gene": "UniProtKB:P82094"
}